{
  "gene_symbol": "AGO3",
  "gene_name": "Protein argonaute-3",
  "gene": "UniProtKB:Q9H9G7",
  "term_id": "GO:0035198",
  "term_label": "miRNA binding"
}